{
  "term_label": "chloride ion homeostasis",
  "gene_symbol": "SLC12A1",
  "term_id": "GO:0055064",
  "gene_name": "Solute carrier family 12 member 1",
  "gene": "UniProtKB:Q13621"
}